biphenyl 2,3-dioxygenase activity [GO:0018687] (molecular function) Relationships: is a type of GO:0016708 Sources: EC:1.14.12.18 Definition: Catalysis of the reaction: biphenyl + NADH + H+ + O2 = (2R,3S)-3-phenylcyclohexa-3,5-diene-1,2-diol + NAD+. This reaction requires Fe2+. Also known as: biphenyl dioxygenase activity, biphenyl,NADH:oxygen oxidoreductase (2,3-hydroxylating)